tetrachloroethylene catabolic process [GO:0019337] (BP) Definition: The chemical reactions and pathways resulting in the breakdown of tetrachloroethylene, a derivative of ethene with the hydrogen atoms replaced by chlorines. References: PMID:7988892, PMID:8663199 Sources: GOC:ai Also known as: tetrachloroethene catabolic process, tetrachloroethene catabolism, tetrachloroethylene breakdown, tetrachloroethylene catabolism, tetrachloroethylene degradation Relationships: is a type of chlorinated hydrocarbon catabolic process [GO:0042205]